{
  "term_id": "GO:0061631",
  "gene_symbol": "UBE2G2",
  "gene_name": "Ubiquitin-conjugating enzyme E2 G2",
  "term_label": "ubiquitin conjugating enzyme activity",
  "gene": "UniProtKB:P60604"
}